{
  "term_label": "GABA-A receptor complex",
  "gene_name": "Gamma-aminobutyric acid receptor subunit alpha-6",
  "gene": "UniProtKB:Q16445",
  "term_id": "GO:1902711",
  "gene_symbol": "GABRA6"
}